{
  "term_id": "GO:0044877",
  "term_label": "protein-containing complex binding",
  "gene": "UniProtKB:Q16795",
  "gene_name": "NADH dehydrogenase [ubiquinone] 1 alpha subcomplex subunit 9, mitochondrial",
  "gene_symbol": "NDUFA9"
}